{
  "gene_symbol": "ELOVL7",
  "term_id": "GO:0034625",
  "gene_name": "Elongation of very long chain fatty acids protein 7",
  "gene": "UniProtKB:A1L3X0",
  "term_label": "fatty acid elongation, monounsaturated fatty acid"
}